{
  "gene_symbol": "C6orf141",
  "term_label": "Unknown cellular component",
  "term_id": "UNKNOWN:0003",
  "gene_name": "Uncharacterized protein C6orf141",
  "gene": "UniProtKB:Q5SZD1"
}